late endosome membrane [GO:0031902] (cellular component) Relationships: is a type of endosome membrane [GO:0010008]; is part of late endosome [GO:0005770] Subtypes: GO:0032585 Definition: The lipid bilayer surrounding a late endosome. Sources: GOC:pz